{
  "gene": "UniProtKB:P29400",
  "term_id": "GO:0030198",
  "term_label": "extracellular matrix organization",
  "gene_symbol": "COL4A5",
  "gene_name": "Collagen alpha-5(IV) chain"
}